{
  "term_id": "GO:0016019",
  "gene_symbol": "PGLYRP4",
  "term_label": "peptidoglycan immune receptor activity",
  "gene": "UniProtKB:Q96LB8",
  "gene_name": "Peptidoglycan recognition protein 4"
}